{
  "gene_name": "HLA class II histocompatibility antigen gamma chain",
  "gene_symbol": "CD74",
  "term_id": "GO:0009986",
  "gene": "UniProtKB:P04233",
  "term_label": "cell surface"
}